metanephric smooth muscle tissue development [GO:0072208] (biological process) Definition: The process whose specific outcome is the progression of smooth muscle in the metanephros over time, from its formation to the mature structure. Sources: GOC:mtg_kidney_jan10 Relationships: is a type of kidney smooth muscle tissue development [GO:0072194]; is part of metanephros development [GO:0001656]